{
  "gene_symbol": "TMX2",
  "term_id": "GO:0005789",
  "term_label": "endoplasmic reticulum membrane",
  "gene_name": "Thioredoxin-related transmembrane protein 2",
  "gene": "UniProtKB:Q9Y320"
}